{
  "gene_symbol": "CDH17",
  "term_id": "GO:0000902",
  "term_label": "cell morphogenesis",
  "gene_name": "Cadherin-17",
  "gene": "UniProtKB:Q12864"
}